{
  "gene": "UniProtKB:O95965",
  "term_id": "GO:0007229",
  "gene_symbol": "ITGBL1",
  "gene_name": "Integrin beta-like protein 1",
  "term_label": "integrin-mediated signaling pathway"
}